ATP-dependent polydeoxyribonucleotide 5'-hydroxyl-kinase activity [GO:0046404] (molecular function) Also known as: polydeoxyribonucleotide 5'-hydroxyl-kinase activity, ATP-dependent DNA kinase activity Sources: RHEA:15669 Relationships: is a type of ATP-dependent polynucleotide 5'-hydroxyl-kinase activity [GO:0051734] Definition: Catalysis of the reaction: ATP + 5'-dephospho-DNA = ADP + 5'-phospho-DNA.